{
  "gene_symbol": "PTTG1IP",
  "gene_name": "Pituitary tumor-transforming gene 1 protein-interacting protein",
  "term_label": "nucleus",
  "gene": "UniProtKB:P53801",
  "term_id": "GO:0005634"
}